{
  "gene_symbol": "P2RX6",
  "term_label": "calcium ion transmembrane transport",
  "gene_name": "P2X purinoceptor 6",
  "term_id": "GO:0070588",
  "gene": "UniProtKB:O15547"
}